cis-acting DNA replication termination [GO:0071946] (BP) Relationships: is a type of site-specific DNA replication termination [GO:0071170] References: PMID:20850009 Sources: GOC:vw Definition: A DNA replication termination process that is initiated by protein binding to a binding site on the same chromosome, but remote from the termination site, via DNA looping or chromosome kissing. Also known as: cis acting DNA replication termination